{
  "term_label": "regulation of heart rate by cardiac conduction",
  "gene_name": "Potassium voltage-gated channel subfamily E member 2",
  "term_id": "GO:0086091",
  "gene_symbol": "KCNE2",
  "gene": "UniProtKB:Q9Y6J6"
}